(S)-3-hydroxyacid-ester dehydrogenase activity [GO:0047109] (molecular function) Note: Note that this term was EC:1.2.1.56. Also known as: (S)-3-hydroxyacid ester dehydrogenase activity, 3-oxo ester (S)-reductase activity, ethyl-(S)-3-hydroxyhexanoate:NADP+ 3-oxidoreductase activity Sources: EC:1.1.1.280, RHEA:18269 Definition: Catalysis of the reaction: ethyl (S)-3-hydroxyhexanoate + NADP+ = ethyl 3-oxohexanoate + H+ + NADPH. Relationships: is a type of oxidoreductase activity, acting on the CH-OH group of donors, NAD or NADP as acceptor [GO:0016616]